pre-miRNA binding [GO:0070883] (molecular function) Relationships: is a type of GO:0003723 References: PMID:18951094 Subtypes: trans-activation response element binding [GO:1990970] Definition: Binding to a precursor microRNA (pre-miRNA) transcript, a stem-loop-containing precursor of microRNA. Also known as: pre-microRNA binding, precursor microRNA binding